repair of kinetochore microtubule attachment defect [GO:0140274] (biological process) Subtypes: repair of mitotic kinetochore microtubule attachment defect [GO:0140273], regulation of spindle attachment to meiosis I kinetochore [GO:1904967] Definition: The cell cycle process where kinetochore microtubule attachment defects are corrected. Relationships: is a type of cell cycle process [GO:0022402] References: PMID:15525536 Also known as: correction of kinetochore microtubule attachment defects, repair of kinetochore microtubule attachment defects